cellular response to macrophage colony-stimulating factor stimulus [GO:0036006] (BP) Definition: Any process that results in a change in state or activity of a cell (in terms of movement, secretion, enzyme production, gene expression, etc.) as a result of a macrophage colony-stimulating factor stimulus. Regulation: regulated by regulation of cellular response to macrophage colony-stimulating factor stimulus [GO:1903972]; negatively regulated by negative regulation of cellular response to macrophage colony-stimulating factor stimulus [GO:1903973]; positively regulated by GO:1903974 Relationships: is a type of response to macrophage colony-stimulating factor [GO:0036005]; is a type of GO:0071345 References: PMID:14687666 Sources: GOC:yaf Also known as: cellular response to M-CSF stimulus, cellular response to macrophage colony-stimulating factor